{
  "term_id": "GO:0000422",
  "term_label": "autophagy of mitochondrion",
  "gene": "UniProtKB:Q9NT62",
  "gene_name": "Ubiquitin-like-conjugating enzyme ATG3",
  "gene_symbol": "ATG3"
}